inner dynein arm assembly [GO:0036159] (biological process) Also known as: IDA assembly Relationships: is a type of GO:0070286 References: PMID:19944400 Sources: GOC:BHF, GOC:vk Definition: The aggregation, arrangement and bonding together of a set of components to form an axonemal dynein inner arm, an inner arm structure present on the outer doublet microtubules of ciliary and flagellar axonemes.